negative regulation of endothelial cell chemotaxis to fibroblast growth factor [GO:2000545] (biological process) Sources: GOC:obol Definition: Any process that stops, prevents or reduces the frequency, rate or extent of endothelial cell chemotaxis to fibroblast growth factor. Relationships: is a type of negative regulation of cell chemotaxis to fibroblast growth factor [GO:1904848]; is a type of regulation of endothelial cell chemotaxis to fibroblast growth factor [GO:2000544]; is a type of negative regulation of endothelial cell chemotaxis [GO:2001027]; negatively regulates endothelial cell chemotaxis to fibroblast growth factor [GO:0035768]